{
  "gene_symbol": "R3HDM4",
  "gene_name": "R3H domain-containing protein 4",
  "term_label": "Unknown cellular component",
  "term_id": "UNKNOWN:0003",
  "gene": "UniProtKB:Q96D70"
}